{
  "term_label": "signaling receptor binding",
  "term_id": "GO:0005102",
  "gene_name": "Na(+)_H(+) exchange regulatory cofactor NHE-RF1",
  "gene_symbol": "NHERF1",
  "gene": "UniProtKB:O14745"
}